{
  "gene_name": "Basic leucine zipper transcriptional factor ATF-like 2",
  "gene_symbol": "BATF2",
  "term_id": "GO:0005634",
  "term_label": "nucleus",
  "gene": "UniProtKB:Q8N1L9"
}